{
  "gene_symbol": "ZIC5",
  "term_label": "RNA polymerase II cis-regulatory region sequence-specific DNA binding",
  "term_id": "GO:0000978",
  "gene": "UniProtKB:Q96T25",
  "gene_name": "Zinc finger protein ZIC 5"
}